{
  "gene_symbol": "PLCB2",
  "term_label": "phosphatidylinositol-4,5-bisphosphate phospholipase C activity",
  "gene": "UniProtKB:Q00722",
  "gene_name": "1-phosphatidylinositol 4,5-bisphosphate phosphodiesterase beta-2",
  "term_id": "GO:0004435"
}